{
  "gene": "UniProtKB:Q9Y485",
  "gene_symbol": "DMXL1",
  "gene_name": "DmX-like protein 1",
  "term_id": "UNKNOWN:0001",
  "term_label": "Unknown molecular function"
}